{
  "gene_name": "Protocadherin-17",
  "term_id": "GO:0050839",
  "term_label": "cell adhesion molecule binding",
  "gene_symbol": "PCDH17",
  "gene": "UniProtKB:O14917"
}